{
  "gene": "UniProtKB:Q9H6Z9",
  "gene_name": "Prolyl hydroxylase EGLN3",
  "term_id": "GO:0005737",
  "term_label": "cytoplasm",
  "gene_symbol": "EGLN3"
}